{
  "gene": "UniProtKB:Q8IZ69",
  "gene_symbol": "TRMT2A",
  "term_label": "Unknown cellular component",
  "gene_name": "tRNA (uracil-5-)-methyltransferase homolog A",
  "term_id": "UNKNOWN:0003"
}